{
  "gene_name": "Zinc finger protein 655",
  "term_label": "DNA-binding transcription factor activity, RNA polymerase II-specific",
  "gene": "UniProtKB:Q8N720",
  "term_id": "GO:0000981",
  "gene_symbol": "ZNF655"
}